{
  "gene": "UniProtKB:Q92613",
  "term_id": "GO:0005634",
  "gene_symbol": "JADE3",
  "gene_name": "Protein Jade-3",
  "term_label": "nucleus"
}